{
  "gene_name": "DNA-binding protein SATB1",
  "term_label": "regulation of transcription by RNA polymerase II",
  "gene_symbol": "SATB1",
  "gene": "UniProtKB:Q01826",
  "term_id": "GO:0006357"
}